{
  "gene_symbol": "CALHM3",
  "gene": "UniProtKB:Q86XJ0",
  "gene_name": "Calcium homeostasis modulator protein 3",
  "term_id": "GO:0005886",
  "term_label": "plasma membrane"
}